anterior lateral line neuromast primordium migration [GO:0048900] (biological process) Relationships: is a type of neuromast primordium migration [GO:0048883]; is part of anterior lateral line development [GO:0048899] References: PMID:15832385 Sources: GOC:dgh Definition: The migration of a cluster of a relatively undifferentiated cell along the developing anterior lateral line, originating from cranial ectodermal placodes situated between the eye and the ear. The neuromast primordium deposits proneuromasts along the lateral line, from which the neuromasts will develop. Also known as: ALL neuromast primordium migration